{
  "gene": "UniProtKB:O43361",
  "term_label": "DNA-binding transcription factor activity, RNA polymerase II-specific",
  "gene_symbol": "ZNF749",
  "gene_name": "Zinc finger protein 749",
  "term_id": "GO:0000981"
}